{
  "gene": "UniProtKB:Q08050",
  "gene_name": "Forkhead box protein M1",
  "term_label": "nucleus",
  "term_id": "GO:0005634",
  "gene_symbol": "FOXM1"
}